{
  "term_id": "UNKNOWN:0002",
  "term_label": "Unknown biological process",
  "gene_symbol": "LINC00052",
  "gene_name": "Putative uncharacterized protein encoded by LINC00052",
  "gene": "UniProtKB:Q96N35"
}